{
  "term_id": "GO:0043138",
  "term_label": "3'-5' DNA helicase activity",
  "gene_symbol": "BLM",
  "gene": "UniProtKB:P54132",
  "gene_name": "RecQ-like DNA helicase BLM"
}